{
  "term_label": "vitamin B6 metabolic process",
  "term_id": "GO:0042816",
  "gene": "UniProtKB:O94903",
  "gene_symbol": "PLPBP",
  "gene_name": "Pyridoxal phosphate homeostasis protein"
}